{
  "gene_symbol": "TRA2B",
  "term_id": "GO:0000398",
  "gene": "UniProtKB:P62995",
  "term_label": "mRNA splicing, via spliceosome",
  "gene_name": "Transformer-2 protein homolog beta"
}